negative regulation of protein localization to cell cortex [GO:1904777] (biological process) Definition: Any process that stops, prevents or reduces the frequency, rate or extent of protein localization to cell cortex. Note: An example is cye-1 in C. elegans, UniProt ID O01501 in PMID:17115027. Subtypes: negative regulation of protein localization to medial cortex [GO:0140325], negative regulation of protein localization to actin cortical patch [GO:1904371] Also known as: down regulation of protein localisation to cell cortex, down regulation of protein localization to cell cortex, down-regulation of protein localisation to cell cortex, down-regulation of protein localization to cell cortex, downregulation of protein localisation to cell cortex, downregulation of protein localization to cell cortex, negative regulation of protein localisation to cell cortex, inhibition of protein localisation to cell cortex, inhibition of protein localization to cell cortex References: PMID:17115027 Sources: GOC:TermGenie, GO_REF:0000058 Relationships: is a type of negative regulation of protein localization to cell periphery [GO:1904376]; is a type of regulation of protein localization to cell cortex [GO:1904776]; negatively regulates protein localization to cell cortex [GO:0072697]